hydrolase activity, acting on carbon-nitrogen (but not peptide) bonds, in nitriles [GO:0016815] (molecular function) Subtypes: nitrilase activity [GO:0000257], thiocyanate hydrolase activity [GO:0018760] Relationships: is a type of GO:0016810 Definition: Catalysis of the hydrolysis of any non-peptide carbon-nitrogen bond in a nitrile, a compound containing the cyano radical, -CN. Sources: GOC:curators